inositol hexakisphosphate binding [GO:0000822] (MF) Also known as: IP6 binding, InsP6 binding Definition: Binding to inositol hexakisphosphate. Relationships: is a type of anion binding [GO:0043168]; is a type of alcohol binding [GO:0043178] Sources: GOC:go_curators